{
  "gene": "UniProtKB:Q8IYT8",
  "term_id": "GO:0005776",
  "term_label": "autophagosome",
  "gene_symbol": "ULK2",
  "gene_name": "Serine_threonine-protein kinase ULK2"
}